{
  "gene_name": "Protocadherin alpha-9",
  "term_label": "cell adhesion molecule binding",
  "gene_symbol": "PCDHA9",
  "term_id": "GO:0050839",
  "gene": "UniProtKB:Q9Y5H5"
}